{
  "term_id": "GO:0051015",
  "gene": "UniProtKB:Q96KX2",
  "term_label": "actin filament binding",
  "gene_name": "F-actin-capping protein subunit alpha-3",
  "gene_symbol": "CAPZA3"
}